DNA metabolic process [GO:0006259] (biological process) Subtypes: telomere maintenance [GO:0000723], GO:0000729, DNA strand displacement [GO:0000732], GO:0000735, formation of extrachromosomal circular DNA [GO:0001325], DNA replication [GO:0006260], GO:0006265, GO:0006270, DNA replication termination [GO:0006274], DNA repair [GO:0006281], base-excision repair, AP site formation [GO:0006285], base-excision repair, gap-filling [GO:0006287], GO:0006297, DNA damage tolerance [GO:0006301], DNA modification [GO:0006304], DNA catabolic process [GO:0006308], DNA recombination [GO:0006310], GO:0015074, DNA strand elongation [GO:0022616], GO:0030491, mitochondrial DNA metabolic process [GO:0032042], GO:0033258, DNA replication, Okazaki fragment processing [GO:0033567], meiotic DNA double-strand break formation [GO:0042138], GO:0042148, DNA protection [GO:0042262], maintenance of DNA repeat elements [GO:0043570], DNA-templated DNA replication maintenance of fidelity [GO:0045005], gap filling involved in double-strand break repair via nonhomologous end joining [GO:0061674], GO:0071139, DNA biosynthetic process [GO:0071897], G-quadruplex DNA formation [GO:0071919], GO:0090629, DNA strand resection involved in replication fork processing [GO:0110025], chromosomal 5-methylcytosine DNA demethylation pathway [GO:0141166] Relationships: is a type of nucleic acid metabolic process [GO:0090304] Definition: Any cellular metabolic process involving deoxyribonucleic acid. This is one of the two main types of nucleic acid, consisting of a long, unbranched macromolecule formed from one, or more commonly, two, strands of linked deoxyribonucleotides. Regulation: regulated by regulation of DNA metabolic process [GO:0051052]; negatively regulated by negative regulation of DNA metabolic process [GO:0051053]; positively regulated by positive regulation of DNA metabolic process [GO:0051054] Also known as: DNA metabolism, cellular DNA metabolism Sources: ISBN:0198506732